ganglioside GP1c binding [GO:1905577] (molecular function) References: PMID:1454804 Sources: GOC:TermGenie, GO_REF:0000067 Definition: Binding to ganglioside GP1c. Relationships: is a type of carboxylic acid binding [GO:0031406]; is a type of ganglioside binding [GO:0035594]